{
  "gene_symbol": "SMIM34",
  "gene_name": "Small integral membrane protein 34",
  "term_label": "Unknown biological process",
  "term_id": "UNKNOWN:0002",
  "gene": "UniProtKB:A8MWV9"
}